{
  "term_label": "melanosome",
  "gene": "UniProtKB:P51159",
  "gene_name": "Ras-related protein Rab-27A",
  "gene_symbol": "RAB27A",
  "term_id": "GO:0042470"
}